{
  "gene_symbol": "GAGE6",
  "term_id": "UNKNOWN:0001",
  "term_label": "Unknown molecular function",
  "gene": "UniProtKB:Q13070",
  "gene_name": "G antigen 6"
}